{
  "term_label": "Unknown cellular component",
  "gene_name": "Immunoglobulin heavy variable 1_OR15-9 (non-functional) (Fragment)",
  "gene_symbol": "IGHV1OR15-9",
  "gene": "UniProtKB:A0A0B4J2B8",
  "term_id": "UNKNOWN:0003"
}